UDP-arabinopyranose mutase activity [GO:0052691] (molecular function) Definition: Catalysis of the reaction: UDP-beta-L-arabinofuranose = UDP-beta-L-arabinopyranose. Relationships: is a type of intramolecular transferase activity [GO:0016866] Sources: EC:5.4.99.30, RHEA:28350 Also known as: UDP-arabinopyranose pyranomutase activity, UDP-L-Ara mutase activity, UDP-L-arabinopyranose furanomutase activity, UDP-L-arabinose mutase activity, uridine-diphosphate-L-arabinose mutase activity